{
  "term_id": "GO:0004648",
  "gene": "UniProtKB:Q9Y617",
  "term_label": "O-phospho-L-serine:2-oxoglutarate aminotransferase activity",
  "gene_symbol": "PSAT1",
  "gene_name": "Phosphoserine aminotransferase"
}